{
  "term_id": "GO:0007189",
  "gene_name": "Adenylate cyclase type 2",
  "gene_symbol": "ADCY2",
  "gene": "UniProtKB:Q08462",
  "term_label": "adenylate cyclase-activating G protein-coupled receptor signaling pathway"
}